symbiont-mediated perturbation of host autophagy [GO:0075071] (biological process) Definition: A process in which a symbiont alters or subverts autophagy in the host cell. The host is defined as the larger of the organisms involved in a symbiotic interaction. Relationships: is a type of GO:0044068 Sources: GOC:pamgo_curators Subtypes: symbiont-mediated activation of host autophagy [GO:0039520], symbiont-mediated suppression of host autophagy [GO:0140321] Also known as: modulation by symbiont of host autophagy, symbiont-mediated modulation of host autophagy, autophagy during symbiotic interaction, autophagy involved in symbiotic interaction, modulation by symbiont of host autophagic process